{
  "term_id": "GO:0005615",
  "term_label": "extracellular space",
  "gene_name": "T-cell surface glycoprotein CD1c",
  "gene_symbol": "CD1C",
  "gene": "UniProtKB:P29017"
}